{
  "gene": "UniProtKB:Q13769",
  "gene_symbol": "THOC5",
  "term_id": "GO:0003729",
  "gene_name": "THO complex subunit 5 homolog",
  "term_label": "mRNA binding"
}